embryonic heart tube elongation [GO:0036306] (BP) Relationships: is a type of anatomical structure development [GO:0048856]; is part of embryonic heart tube development [GO:0035050] References: PMID:15901664 Sources: GOC:BHF, GOC:gr Definition: The developmental growth that results in the increase in length of the embryonic heart tube. The embryonic heart tube is an epithelial tube that will give rise to the mature heart.